{
  "gene": "UniProtKB:Q8IYD8",
  "gene_symbol": "FANCM",
  "gene_name": "Fanconi anemia group M protein",
  "term_label": "interstrand cross-link repair",
  "term_id": "GO:0036297"
}